axon development [GO:0061564] (biological process) Relationships: is_a neuron projection development [GO:0031175] Subtypes: GO:0031103, afferent axon development in lateral line nerve [GO:0048893] Definition: The progression of an axon over time. Covers axonogenesis (de novo generation of an axon) and axon regeneration (regrowth), as well as processes pertaining to the progression of the axon over time (fasciculation and defasciculation). Sources: GOC:dph, GOC:pg, GOC:pr